{
  "term_id": "GO:0003823",
  "term_label": "antigen binding",
  "gene_name": "Immunoglobulin heavy variable 1-46",
  "gene": "UniProtKB:P01743",
  "gene_symbol": "IGHV1-46"
}